{
  "gene_name": "Adapter molecule crk",
  "gene": "UniProtKB:P46108",
  "gene_symbol": "CRK",
  "term_id": "GO:0016477",
  "term_label": "cell migration"
}